{
  "gene": "UniProtKB:P49711",
  "term_id": "GO:0003700",
  "term_label": "DNA-binding transcription factor activity",
  "gene_symbol": "CTCF",
  "gene_name": "Transcriptional repressor CTCF"
}